reduction of food intake in response to dietary excess [GO:0002023] (BP) Definition: An eating behavior process whereby detection of a dietary excess results in a decrease in intake of nutrients. References: PMID:12161655, PMID:12840200 Sources: GOC:pg, GOC:pr Relationships: is a type of eating behavior [GO:0042755]; is part of response to dietary excess [GO:0002021]